{
  "gene_symbol": "FAXDC2",
  "term_label": "sterol biosynthetic process",
  "term_id": "GO:0016126",
  "gene": "UniProtKB:Q96IV6",
  "gene_name": "Fatty acid hydroxylase domain-containing protein 2"
}